{
  "term_id": "UNKNOWN:0001",
  "gene_symbol": "IFT122",
  "term_label": "Unknown molecular function",
  "gene_name": "Intraflagellar transport protein 122 homolog",
  "gene": "UniProtKB:Q9HBG6"
}